lysosomal lumen acidification [GO:0007042] (biological process) Also known as: lysosome pH reduction Relationships: is a type of GO:0007035; is a type of GO:0035751 Definition: Any process that reduces the pH of the lysosomal lumen, measured by the concentration of the hydrogen ion. Sources: GOC:jid